plasma membrane raft polarization [GO:0044858] (biological process) Also known as: plasma membrane polarization Definition: The clustering and aggregation of a plasma membrane into domains. This serves as a mechanism to compartmentalize cellular activities and to establish cell polarity. Relationships: is a type of membrane raft polarization [GO:0001766]; is a type of plasma membrane raft distribution [GO:0044855] Sources: GOC:jl Regulation: regulated by regulation of plasma membrane raft polarization [GO:1903906]; negatively regulated by negative regulation of plasma membrane raft polarization [GO:1903907]; positively regulated by GO:1903908